{
  "term_id": "GO:0010008",
  "gene_name": "Ras-related protein Rab-23",
  "term_label": "endosome membrane",
  "gene_symbol": "RAB23",
  "gene": "UniProtKB:Q9ULC3"
}